{
  "term_label": "plasma membrane",
  "gene_name": "Olfactory receptor 10G3",
  "gene_symbol": "OR10G3",
  "term_id": "GO:0005886",
  "gene": "UniProtKB:Q8NGC4"
}